skeletal myofibril assembly [GO:0014866] (biological process) Sources: GOC:ef, GOC:mtg_muscle Relationships: is a type of myofibril assembly [GO:0030239] Definition: The process whose specific outcome is the progression of the skeletal myofibril over time, from its formation to the mature structure. A skeletal myofibril is a myofibril specific to skeletal muscle cells.